{
  "term_label": "myosin II complex",
  "gene": "UniProtKB:P35579",
  "term_id": "GO:0016460",
  "gene_symbol": "MYH9",
  "gene_name": "Myosin-9"
}